{
  "term_label": "RNA polymerase II cis-regulatory region sequence-specific DNA binding",
  "gene_name": "Interferon regulatory factor 9",
  "gene": "UniProtKB:Q00978",
  "gene_symbol": "IRF9",
  "term_id": "GO:0000978"
}